telomere-telomerase complex [GO:0070565] (cellular component) Note: Note that this term can be used in place of the obsolete cellular component term 'telomere ; GO:0005696'. Use with caution because this term refers to a specific protein complex and not a region of the chromosome. Definition: A complex of DNA and protein located at the end of a linear chromosome that enables replication of the telomeric repeat sequences at the end of a linear chromosome. Relationships: is a type of protein-DNA complex [GO:0032993]; is part of chromosome, telomeric region [GO:0000781] References: PMID:19179534 Sources: GOC:pde